{
  "term_label": "regulation of transcription by RNA polymerase II",
  "term_id": "GO:0006357",
  "gene": "UniProtKB:Q02577",
  "gene_symbol": "NHLH2",
  "gene_name": "Helix-loop-helix protein 2"
}